{
  "gene_name": "Intracellular hyaluronan-binding protein 4",
  "gene_symbol": "HABP4",
  "term_label": "nucleus",
  "gene": "UniProtKB:Q5JVS0",
  "term_id": "GO:0005634"
}